{
  "term_label": "cell-cell adhesion mediator activity",
  "gene_symbol": "NEXN",
  "gene_name": "Nexilin",
  "gene": "UniProtKB:Q0ZGT2",
  "term_id": "GO:0098632"
}